positive regulation of ammonia assimilation cycle [GO:2001250] (biological process) Also known as: positive regulation of glutamate metabolic process via glutamine and ammonia, positive regulation of glutamate metabolism via glutamine and ammonia Sources: GOC:BHF Relationships: is a type of positive regulation of amino acid metabolic process [GO:0045764]; is_a positive regulation of nitrogen utilization [GO:0045848]; is a type of positive regulation of small molecule metabolic process [GO:0062013]; is a type of GO:2001248; positively regulates ammonia assimilation cycle [GO:0019676] Definition: Any process that activates or increases the frequency, rate or extent of ammonia assimilation cycle.